{
  "gene_symbol": "ZNF444",
  "term_id": "UNKNOWN:0003",
  "gene": "UniProtKB:Q8N0Y2",
  "gene_name": "Zinc finger protein 444",
  "term_label": "Unknown cellular component"
}